inositol-1,4,5,6-tetrakisphosphate 6-phosphatase activity [GO:0030352] (molecular function) Relationships: is a type of inositol tetrakisphosphate phosphatase activity [GO:0052743] Definition: Catalysis of the reaction: 1D-myo-inositol 1,4,5,6-tetrakisphosphate + H2O = 1D-myo-inositol 1,4,5-trisphosphate + phosphate. Sources: RHEA:77147